{
  "term_id": "GO:0000981",
  "gene_symbol": "ZNF625",
  "gene_name": "Zinc finger protein 625",
  "term_label": "DNA-binding transcription factor activity, RNA polymerase II-specific",
  "gene": "UniProtKB:Q96I27"
}